{
  "gene_symbol": "UBE2M",
  "gene_name": "NEDD8-conjugating enzyme Ubc12",
  "term_label": "NEDD8 transferase activity",
  "gene": "UniProtKB:P61081",
  "term_id": "GO:0019788"
}